{
  "term_label": "chromatin binding",
  "term_id": "GO:0003682",
  "gene_name": "Protein STPG4",
  "gene_symbol": "STPG4",
  "gene": "UniProtKB:Q8N801"
}